{
  "gene_name": "Solute carrier family 22 member 12",
  "term_label": "Unknown cellular component",
  "gene": "UniProtKB:Q96S37",
  "gene_symbol": "SLC22A12",
  "term_id": "UNKNOWN:0003"
}